{
  "gene_symbol": "RPL37",
  "term_id": "UNKNOWN:0002",
  "term_label": "Unknown biological process",
  "gene": "UniProtKB:P61927",
  "gene_name": "Large ribosomal subunit protein eL37"
}